{
  "term_label": "long-chain fatty acid biosynthetic process",
  "gene_symbol": "ACSBG2",
  "gene": "UniProtKB:Q5FVE4",
  "term_id": "GO:0042759",
  "gene_name": "Long-chain-fatty-acid--CoA ligase ACSBG2"
}